{
  "gene": "UniProtKB:Q96RD9",
  "gene_symbol": "FCRL5",
  "term_id": "GO:0009897",
  "gene_name": "Fc receptor-like protein 5",
  "term_label": "external side of plasma membrane"
}